{
  "gene": "UniProtKB:Q9UQ84",
  "gene_name": "Exonuclease 1",
  "term_label": "5'-3' DNA exonuclease activity",
  "gene_symbol": "EXO1",
  "term_id": "GO:0035312"
}